{
  "gene": "UniProtKB:Q86WS4",
  "gene_symbol": "C12orf40",
  "term_id": "UNKNOWN:0002",
  "term_label": "Unknown biological process",
  "gene_name": "Uncharacterized protein C12orf40"
}